{
  "term_label": "cytoplasm",
  "gene_symbol": "DRG1",
  "term_id": "GO:0005737",
  "gene_name": "Developmentally-regulated GTP-binding protein 1",
  "gene": "UniProtKB:Q9Y295"
}